{
  "gene": "UniProtKB:M5A8F1",
  "term_id": "UNKNOWN:0002",
  "gene_symbol": "ERVH48-1",
  "gene_name": "Suppressyn",
  "term_label": "Unknown biological process"
}